regulation of establishment of cell polarity [GO:2000114] (biological process) Definition: Any process that modulates the frequency, rate or extent of establishment of cell polarity. Also known as: regulation of cell polarization, regulation of bud site selection/establishment of cell polarity Sources: GOC:dph Relationships: is a type of GO:0032878; regulates GO:0030010 Subtypes: regulation of establishment of bipolar cell polarity [GO:0061172], GO:1903903, regulation of establishment of cell polarity regulating cell shape [GO:2000782]